{
  "term_label": "endoplasmic reticulum signal peptide binding",
  "gene_name": "Signal recognition particle subunit SRP54",
  "gene": "UniProtKB:P61011",
  "term_id": "GO:0030942",
  "gene_symbol": "SRP54"
}